{
  "gene_name": "Down syndrome critical region protein 4",
  "gene": "UniProtKB:P56555",
  "gene_symbol": "DSCR4",
  "term_id": "UNKNOWN:0001",
  "term_label": "Unknown molecular function"
}